{
  "gene": "UniProtKB:P41271",
  "term_id": "GO:0036122",
  "term_label": "BMP binding",
  "gene_symbol": "NBL1",
  "gene_name": "Neuroblastoma suppressor of tumorigenicity 1"
}